regulation of embryo sac egg cell differentiation [GO:0045694] (biological process) Also known as: regulation of female gametophyte egg cell differentiation Definition: Any process that modulates the frequency, rate or extent of embryo sac egg cell differentiation. Sources: GOC:go_curators, GOC:mtg_plant Subtypes: GO:0045695, positive regulation of embryo sac egg cell differentiation [GO:0045696] Relationships: is a type of regulation of cell differentiation [GO:0045595]; is a type of regulation of reproductive process [GO:2000241]; regulates GO:0009560